{
  "term_label": "Golgi cis cisterna",
  "gene_name": "Golgin subfamily A member 6B",
  "gene": "UniProtKB:A6NDN3",
  "term_id": "GO:0000137",
  "gene_symbol": "GOLGA6B"
}